ferredoxin hydrogenase activity [GO:0008901] (molecular function) Sources: EC:1.12.7.2 Relationships: is a type of oxidoreductase activity, acting on hydrogen as donor, iron-sulfur protein as acceptor [GO:0016699] Also known as: H(2) oxidizing hydrogenase activity, H(2) producing hydrogenase activity, H2 oxidizing hydrogenase, H2 producing hydrogenase, bidirectional hydrogenase activity, hydrogen-lyase activity, hydrogenase activity, hydrogenlyase activity, uptake hydrogenase activity, [Fe] hydrogenase activity, hydrogen:ferredoxin oxidoreductase activity, Ni-Fe hydrogenase activity, Ni-Fe-Se hydrogenase activity, iron hydrogenase activity, iron-only hydrogenase activity, nickel hydrogenase activity, nickel-iron hydrogenase activity, nickel-iron-selenium hydrogenase activity, [Fe] hydrogenase gamma, hydrogenase (ferredoxin) activity, hydrogenase I, hydrogenase II Definition: Catalysis of the reaction: 2 reduced ferredoxin + 2 H+ = 2 oxidized ferredoxin + H2.